{
  "term_id": "GO:0008188",
  "term_label": "neuropeptide receptor activity",
  "gene_symbol": "NMBR",
  "gene": "UniProtKB:P28336",
  "gene_name": "Neuromedin-B receptor"
}